cellular response to redox state [GO:0071461] (biological process) Also known as: cellular redox signal response Sources: GOC:mah Relationships: is a type of response to redox state [GO:0051775] Definition: Any process that results in a change in state or activity of a cell (in terms of movement, secretion, enzyme production, gene expression, etc.) as a result of a stimulus indicating redox state. Redox state refers to the balance of oxidized versus reduced forms of electron donors and acceptors in an organelle, cell or organ; plastoquinone, glutathione (GSH/GSSG), and nicotinamide nucleotides (NAD+/NADH and NADP+/NADPH) are among the most important.